{
  "gene": "UniProtKB:Q13151",
  "term_label": "3'-UTR-mediated mRNA stabilization",
  "gene_symbol": "HNRNPA0",
  "term_id": "GO:0070935",
  "gene_name": "Heterogeneous nuclear ribonucleoprotein A0"
}